response to dextromethorphan [GO:1904558] (biological process) Relationships: is a type of GO:0014072; is a type of response to ether [GO:0045472] References: PMID:25796330 Sources: GOC:TermGenie, GOC:mr, GO_REF:0000071 Definition: Any process that results in a change in state or activity of a cell or an organism (in terms of movement, secretion, enzyme production, gene expression, etc.) as a result of a dextromethorphan stimulus. Subtypes: GO:1904559